positive regulation of protein kinase activity [GO:0045860] (biological process) Subtypes: GO:0032147, positive regulation of protein tyrosine kinase activity [GO:0061098], positive regulation of protein serine/threonine kinase activity [GO:0071902], positive regulation of cyclin-dependent protein kinase activity [GO:1904031] Also known as: up regulation of protein kinase activity, up-regulation of protein kinase activity, upregulation of protein kinase activity, stimulation of protein kinase activity Relationships: is a type of positive regulation of protein phosphorylation [GO:0001934]; is a type of GO:0033674; is a type of GO:0045859; positively regulates protein kinase activity [GO:0004672] Sources: GOC:go_curators Definition: Any process that activates or increases the frequency, rate or extent of protein kinase activity.